diphosphomevalonate decarboxylase activity [GO:0004163] (molecular function) Definition: Catalysis of the reaction: (R)-5-diphosphomevalonate + ATP = ADP + CO2 + H+ + isopentenyl diphosphate + phosphate. Sources: EC:4.1.1.33, RHEA:23732 Also known as: 5-pyrophosphomevalonate decarboxylase activity, ATP:(R)-5-diphosphomevalonate carboxy-lyase (adding ATP; isopentenyl-diphosphate-forming), ATP:(R)-5-diphosphomevalonate carboxy-lyase (dehydrating), mevalonate 5-diphosphate decarboxylase activity, mevalonate diphosphate decarboxylase activity, mevalonate pyrophosphate decarboxylase activity, mevalonate-5-pyrophosphate decarboxylase activity, pyrophosphomevalonate decarboxylase activity, pyrophosphomevalonic acid decarboxylase activity Relationships: is a type of carboxy-lyase activity [GO:0016831]